salivary gland morphogenesis [GO:0007435] (biological process) Subtypes: larval salivary gland morphogenesis [GO:0007436], adult salivary gland morphogenesis [GO:0007437], GO:0035070 Sources: GOC:jid Relationships: is a type of gland morphogenesis [GO:0022612]; is part of salivary gland development [GO:0007431] Definition: The process in which the anatomical structures of the salivary gland are generated and organized. Regulation: positively regulated by positive regulation of salivary gland formation by mesenchymal-epithelial signaling [GO:0060639]